{
  "gene_name": "T-cell leukemia homeobox protein 1",
  "term_label": "regulation of transcription by RNA polymerase II",
  "gene": "UniProtKB:P31314",
  "gene_symbol": "TLX1",
  "term_id": "GO:0006357"
}